{
  "term_label": "Unknown molecular function",
  "term_id": "UNKNOWN:0001",
  "gene_symbol": "BTBD3",
  "gene": "UniProtKB:Q9Y2F9",
  "gene_name": "BTB_POZ domain-containing protein 3"
}